{
  "term_id": "GO:0035249",
  "gene_name": "Vesicular glutamate transporter 3",
  "gene_symbol": "SLC17A8",
  "term_label": "synaptic transmission, glutamatergic",
  "gene": "UniProtKB:Q8NDX2"
}